positive regulation of small GTPase mediated signal transduction [GO:0051057] (biological process) Definition: Any process that activates or increases the frequency, rate or extent of small GTPase mediated signal transduction. Sources: GOC:ai Also known as: positive regulation of small GTPase-mediated signal transduction, up regulation of small GTPase mediated signal transduction, up-regulation of small GTPase mediated signal transduction, upregulation of small GTPase mediated signal transduction, activation of small GTPase mediated signal transduction, stimulation of small GTPase mediated signal transduction Relationships: is a type of regulation of small GTPase mediated signal transduction [GO:0051056]; is a type of positive regulation of intracellular signal transduction [GO:1902533]; positively regulates GO:0007264 Subtypes: positive regulation of septation initiation signaling [GO:0031031], positive regulation of ARF protein signal transduction [GO:0032014], positive regulation of Rac protein signal transduction [GO:0035022], GO:0035025, positive regulation of Ras protein signal transduction [GO:0046579]